{
  "gene_name": "TBC1 domain family member 14",
  "term_label": "GTPase activator activity",
  "gene_symbol": "TBC1D14",
  "term_id": "GO:0005096",
  "gene": "UniProtKB:Q9P2M4"
}